citrate:succinate antiporter activity [GO:0015515] (molecular function) Definition: Enables the transfer of a solute or solutes from one side of a membrane to the other according to the reaction: citrate(out) + succinate(in) = citrate(in) + succinate(out). Relationships: is a type of succinate transmembrane transporter activity [GO:0015141]; is a type of GO:0015297; is a type of citrate secondary active transmembrane transporter activity [GO:0071913] Sources: TC:2.A.47.3.2